{
  "gene": "UniProtKB:Q969S3",
  "gene_name": "Cytoplasmic 60S subunit biogenesis factor ZNF622",
  "term_id": "UNKNOWN:0001",
  "gene_symbol": "ZNF622",
  "term_label": "Unknown molecular function"
}